{
  "term_label": "chitin catabolic process",
  "gene": "UniProtKB:Q12889",
  "term_id": "GO:0006032",
  "gene_name": "Oviduct-specific glycoprotein",
  "gene_symbol": "OVGP1"
}